fatty acid amide hydrolase activity [GO:0017064] (molecular function) Definition: Catalysis of the hydrolysis of a fatty acid amide to yield a fatty acid. Also known as: anandamide amidohydrolase activity, oleamide hydrolase activity References: PMID:15952893 Relationships: is a type of GO:0016811